{
  "term_id": "GO:0005289",
  "gene_symbol": "SLC25A29",
  "term_label": "high-affinity L-arginine transmembrane transporter activity",
  "gene_name": "Mitochondrial basic amino acids transporter",
  "gene": "UniProtKB:Q8N8R3"
}